{
  "gene": "UniProtKB:Q9UIK4",
  "term_id": "GO:0043065",
  "gene_name": "Death-associated protein kinase 2",
  "term_label": "positive regulation of apoptotic process",
  "gene_symbol": "DAPK2"
}